interleukin-27 complex [GO:0070744] (cellular component) Relationships: is a type of protein-containing complex [GO:0032991]; is part of extracellular space [GO:0005615] Definition: A protein complex that is composed of an interleukin-27p28 subunit (product of the IL27 gene) and an EBI3 subunit and is secreted into the extracellular space. References: PMID:15999093, PMID:19161428 Sources: GOC:add Also known as: IL-27 complex, EBI3, IL27, p28 Note: Note that this heterodimeric cytokine utilizes the same EBI3 subunit (product of EBI3, Epstein-Barr virus induced gene 3) as its beta chain as IL-35 uses for its beta chain. Also note that the product of the IL27 gene is the alpha subunit of IL-27. The functional IL-27 protein complex requires both subunits.